regulation of root meristem growth [GO:0010082] (biological process) Also known as: regulation of root meristem size Definition: Any process involved in maintaining the size and shape of a root meristem. Relationships: is a type of regulation of meristem growth [GO:0010075]; is part of root morphogenesis [GO:0010015]; regulates root meristem growth [GO:0010449] Sources: GOC:tb